{
  "term_id": "GO:0098655",
  "gene_name": "Cyclic nucleotide-gated cation channel beta-3",
  "term_label": "monoatomic cation transmembrane transport",
  "gene": "UniProtKB:Q9NQW8",
  "gene_symbol": "CNGB3"
}